{
  "gene_name": "Polyunsaturated fatty acid lipoxygenase ALOX15",
  "term_label": "linoleate 13S-lipoxygenase activity",
  "term_id": "GO:0016165",
  "gene": "UniProtKB:P16050",
  "gene_symbol": "ALOX15"
}